Purkinje myocyte differentiation [GO:0003168] (biological process) Definition: The process in which a relatively unspecialized cell acquires the specialized structural and/or functional features of a Purkinje myocyte (also known as cardiac Purkinje fiber cell). These cells are specialized cardiomyocytes that receive signals from the bundle of His and innervate the ventricular cardiac muscle. Relationships: is_a His-Purkinje system cell differentiation [GO:0060932]; is part of GO:0003165 Also known as: cardiac Purkinje fiber cell differentiation Sources: GOC:mtg_cardiac_conduct_nov11, GOC:mtg_heart